{
  "gene_symbol": "AIMP1",
  "term_label": "Unknown molecular function",
  "term_id": "UNKNOWN:0001",
  "gene_name": "Aminoacyl tRNA synthase complex-interacting multifunctional protein 1",
  "gene": "UniProtKB:Q12904"
}